{
  "term_label": "lysosome",
  "gene": "UniProtKB:Q96AH8",
  "term_id": "GO:0005764",
  "gene_symbol": "RAB7B",
  "gene_name": "Ras-related protein Rab-7b"
}